negative regulation of cellular response to iron ion starvation [GO:1901967] (biological process) Definition: Any process that stops, prevents or reduces the frequency, rate or extent of cellular response to iron ion starvation. Also known as: down regulation of cellular response to iron ion starvation, down-regulation of cellular response to iron ion starvation, downregulation of cellular response to iron ion starvation, inhibition of cellular response to iron ion starvation References: PMID:23115244 Sources: GOC:TermGenie Relationships: is a type of negative regulation of response to nutrient levels [GO:0032108]; is a type of negative regulation of cellular process [GO:0048523]; is a type of GO:1901966; negatively regulates GO:0010106